indole-containing compound metabolic process [GO:0042430] (biological process) Definition: The chemical reactions and pathways involving compounds that contain an indole (2,3-benzopyrrole) skeleton. Also known as: indole and derivative metabolic process, indole and derivative metabolism, indole-containing compound metabolism, ketole metabolic process, ketole metabolism, indole derivative metabolic process, indole derivative metabolism Subtypes: L-tryptophan metabolic process [GO:0006568], GO:0019356, melatonin metabolic process [GO:0030186], GO:0033473, indole glucosinolate metabolic process [GO:0042343], serotonin metabolic process [GO:0042428], indole metabolic process [GO:0042431], indole-containing compound biosynthetic process [GO:0042435], indole-containing compound catabolic process [GO:0042436], indolebutyric acid metabolic process [GO:0080024] Relationships: is a type of GO:0008152 Sources: GOC:jl, GOC:mah